{
  "term_id": "GO:0042824",
  "gene": "UniProtKB:Q03519",
  "gene_symbol": "TAP2",
  "gene_name": "Antigen peptide transporter 2",
  "term_label": "MHC class I peptide loading complex"
}